{
  "term_id": "GO:0042147",
  "term_label": "retrograde transport, endosome to Golgi",
  "gene_name": "Ras-related protein Rab-41",
  "gene_symbol": "RAB41",
  "gene": "UniProtKB:Q5JT25"
}